negative regulation of compound eye retinal cell programmed cell death [GO:0046673] (biological process) Definition: Any process that stops, prevents, or reduces the frequency, rate or extent of programmed cell death that occurs in the compound eye retina. Also known as: down regulation of retinal cell programmed cell death, down-regulation of retinal cell programmed cell death, downregulation of retinal cell programmed cell death, inhibition of retinal cell programmed cell death, negative regulation of retina cell programmed cell death, negative regulation of retinal cell programmed cell death Relationships: is a type of GO:0046669; is a type of negative regulation of retinal cell programmed cell death [GO:0046671]; negatively regulates compound eye retinal cell programmed cell death [GO:0046667] Sources: GOC:ai